interleukin-23 receptor complex [GO:0072536] (cellular component) Relationships: is a type of plasma membrane signaling receptor complex [GO:0098802] Definition: A protein complex that binds interleukin-23 and that consists of, at a minimum, a dimeric interleukin and its two receptor subunits as well as optional additional kinase subunits. Also known as: IL-23 receptor complex References: PMID:12023369 Sources: GOC:BHF, GOC:mah